{
  "gene_name": "Short-chain dehydrogenase_reductase 3",
  "gene_symbol": "DHRS3",
  "term_label": "lipid droplet",
  "gene": "UniProtKB:O75911",
  "term_id": "GO:0005811"
}